protein localization to endoplasmic reticulum tubular network [GO:1903420] (BP) References: PMID:25103238 Sources: GOC:TermGenie, GO_REF:0000087 Relationships: is a type of protein localization to endoplasmic reticulum [GO:0070972] Definition: A process in which a protein is transported to, or maintained in, a location within an endoplasmic reticulum tubular network. Subtypes: protein localization to cortical endoplasmic reticulum [GO:1903419] Also known as: protein localisation in endoplasmic reticulum tubular network, protein localisation to endoplasmic reticulum tubular network, protein localization in endoplasmic reticulum tubular network, protein localization to tubular ER